positive regulation of response to biotic stimulus [GO:0002833] (biological process) Subtypes: positive regulation of antimicrobial humoral response [GO:0002760], positive regulation of response to tumor cell [GO:0002836], positive regulation of lipopolysaccharide-mediated signaling pathway [GO:0031666], positive regulation of innate immune response [GO:0045089], positive regulation of neutrophil mediated killing of symbiont cell [GO:0070961], positive regulation of defense response to insect [GO:1900367], GO:1900426, GO:1900445, positive regulation of systemic acquired resistance [GO:1901672], positive regulation of response to cell cycle checkpoint signaling [GO:1902146], positive regulation of defense response to oomycetes [GO:1902290] Sources: GOC:add Note: Note that this term is in the subset of terms that should not be used for direct gene product annotation. Instead, select a child term or, if no appropriate child term exists, please request a new term. Direct annotations to this term may be amended during annotation QC. Relationships: is a type of GO:0002831; is a type of positive regulation of response to stimulus [GO:0048584]; positively regulates response to biotic stimulus [GO:0009607] Also known as: up regulation of response to biotic stimulus, up-regulation of response to biotic stimulus, upregulation of response to biotic stimulus, activation of response to biotic stimulus, stimulation of response to biotic stimulus Definition: Any process that activates or increases the frequency, rate, or extent of a response to biotic stimulus.